{
  "term_label": "dendrite",
  "gene_symbol": "KLHL1",
  "term_id": "GO:0030425",
  "gene": "UniProtKB:Q9NR64",
  "gene_name": "Kelch-like protein 1"
}